{
  "term_id": "GO:0005615",
  "gene_symbol": "EDA",
  "gene": "UniProtKB:Q92838",
  "term_label": "extracellular space",
  "gene_name": "Ectodysplasin-A"
}